{
  "term_label": "endocytic recycling",
  "gene_name": "Sorting nexin-31",
  "gene": "UniProtKB:Q8N9S9",
  "term_id": "GO:0032456",
  "gene_symbol": "SNX31"
}